positive regulation of connective tissue growth factor production [GO:0032723] (biological process) Relationships: is a type of positive regulation of cytokine production [GO:0001819]; is a type of regulation of connective tissue growth factor production [GO:0032643]; RO_0002213 connective tissue growth factor production [GO:0032601] Sources: GOC:mah Definition: Any process that activates or increases the frequency, rate, or extent of connective tissue growth factor production. Also known as: positive regulation of CCN2 production, positive regulation of CTGF production, positive regulation of Fisp12 production, positive regulation of Hcs24 production, positive regulation of IGFBP8 production, positive regulation of hypertrophic chondrocyte-specific gene product 24 production, up regulation of connective tissue growth factor production, up-regulation of connective tissue growth factor production, upregulation of connective tissue growth factor production, activation of connective tissue growth factor production, positive regulation of connective tissue growth factor biosynthetic process, stimulation of connective tissue growth factor production